{
  "gene_symbol": "OPRM1",
  "term_label": "G-protein beta-subunit binding",
  "gene_name": "Mu-type opioid receptor",
  "term_id": "GO:0031681",
  "gene": "UniProtKB:P35372"
}